{
  "term_label": "membrane",
  "gene_name": "Endoplasmic reticulum mannosyl-oligosaccharide 1,2-alpha-mannosidase",
  "term_id": "GO:0016020",
  "gene": "UniProtKB:Q9UKM7",
  "gene_symbol": "MAN1B1"
}